{
  "gene_name": "Cyclin-dependent kinase 5 activator 1",
  "gene_symbol": "CDK5R1",
  "term_id": "GO:0030426",
  "term_label": "growth cone",
  "gene": "UniProtKB:Q15078"
}